endoplasmic reticulum-plasma membrane tethering [GO:0061817] (biological process) References: PMID:23237950, PMID:26877082, PMID:27875684 Sources: GOC:dph, GOC:vw Also known as: ER-plasma membrane tethering Relationships: is a type of GO:0051643; is a type of GO:0140056 Definition: The attachment of an endoplasmic reticulum membrane to the plasma membrane via molecular tethers.